{
  "gene_name": "Histone H2B type F-S",
  "term_label": "structural constituent of chromatin",
  "gene_symbol": "H2BC12L",
  "term_id": "GO:0030527",
  "gene": "UniProtKB:P57053"
}